T/G mismatch-specific endonuclease activity [GO:0043765] (molecular function) References: PMID:17651368 Definition: Catalysis of the repair of T/G mismatches arising from deamination of 5-methylcytosine in DNA by nicking double-stranded DNA within the sequence CT(AT)GN or NT(AT)GG next to the mismatched thymidine residue. The incision is mismatch-dependent and strand-specific, in favor of the G-containing strand. The incision serves as a starting point for subsequent excision repair by DNA polymerase I, which excises thymidine and reinserts cytidine. Also known as: DNA mismatch endonuclease, V.EcoKDcm, Vsr mismatch endonuclease, very short patch repair protein Relationships: is a type of DNA endonuclease activity [GO:0004520]